{
  "gene_symbol": "ZIC3",
  "gene_name": "Zinc finger protein ZIC 3",
  "term_id": "GO:0007417",
  "gene": "UniProtKB:O60481",
  "term_label": "central nervous system development"
}